{
  "gene": "UniProtKB:P01350",
  "gene_name": "Gastrin",
  "term_label": "response to food",
  "term_id": "GO:0032094",
  "gene_symbol": "GAST"
}